{
  "term_id": "GO:0000978",
  "gene": "UniProtKB:Q3C1V8",
  "gene_name": "Brain-specific homeobox protein homolog",
  "term_label": "RNA polymerase II cis-regulatory region sequence-specific DNA binding",
  "gene_symbol": "BSX"
}